negative regulation of oligodendrocyte apoptotic process [GO:1900142] (biological process) Also known as: down regulation of oligodendrocyte apoptotic process, down-regulation of oligodendrocyte apoptotic process, downregulation of oligodendrocyte apoptotic process, down regulation of oligodendrocyte apoptosis, down-regulation of oligodendrocyte apoptosis, downregulation of oligodendrocyte apoptosis, inhibition of oligodendrocyte apoptosis, inhibition of oligodendrocyte apoptotic process, negative regulation of oligodendrocyte apoptosis Relationships: is a type of negative regulation of glial cell apoptotic process [GO:0034351]; is a type of GO:1900141; RO_0002212 oligodendrocyte apoptotic process [GO:0097252] Sources: GOC:TermGenie, GOC:yaf Definition: Any process that stops, prevents or reduces the frequency, rate or extent of oligodendrocyte apoptotic process.